{
  "gene_symbol": "L1TD1",
  "term_id": "GO:1990904",
  "gene": "UniProtKB:Q5T7N2",
  "term_label": "ribonucleoprotein complex",
  "gene_name": "LINE-1 type transposase domain-containing protein 1"
}